D-xylose catabolic process [GO:0042843] (biological process) Regulation: regulated by GO:0043469 Subtypes: GO:0044577 Sources: ISBN:0198506732 Definition: The chemical reactions and pathways resulting in the breakdown of D-xylose, a naturally occurring plant polysaccharide. Relationships: is a type of GO:0019323; is a type of GO:0042732 Also known as: D-xylose breakdown, D-xylose catabolism, D-xylose degradation